{
  "gene_symbol": "COX15",
  "gene": "UniProtKB:Q7KZN9",
  "term_id": "GO:0120547",
  "gene_name": "Cytochrome c oxidase assembly protein COX15 homolog",
  "term_label": "heme A synthase activity"
}